{
  "gene": "UniProtKB:Q13394",
  "term_label": "Unknown biological process",
  "term_id": "UNKNOWN:0002",
  "gene_symbol": "MAB21L1",
  "gene_name": "Putative nucleotidyltransferase MAB21L1"
}